{
  "term_label": "Unknown molecular function",
  "term_id": "UNKNOWN:0001",
  "gene": "UniProtKB:O14562",
  "gene_symbol": "UBFD1",
  "gene_name": "Ubiquitin domain-containing protein UBFD1"
}